{
  "gene_name": "Notchless protein homolog 1",
  "gene_symbol": "NLE1",
  "term_label": "regulation of Notch signaling pathway",
  "term_id": "GO:0008593",
  "gene": "UniProtKB:Q9NVX2"
}